protein stearoylation [GO:0140438] (biological process) Relationships: is a type of protein lipidation [GO:0006497] Definition: The covalent attachment of a stearoyl group to an amino acid in a protein. References: PMID:26214738